{
  "gene_name": "Complement component 1 Q subcomponent-binding protein, mitochondrial",
  "gene": "UniProtKB:Q07021",
  "term_label": "negative regulation of mRNA splicing, via spliceosome",
  "gene_symbol": "C1QBP",
  "term_id": "GO:0048025"
}